{
  "gene_symbol": "MST1",
  "gene": "UniProtKB:P26927",
  "gene_name": "Hepatocyte growth factor-like protein",
  "term_id": "GO:0046425",
  "term_label": "regulation of receptor signaling pathway via JAK-STAT"
}